{
  "gene": "UniProtKB:P18859",
  "gene_name": "ATP synthase-coupling factor 6, mitochondrial",
  "gene_symbol": "ATP5PF",
  "term_label": "proton-transporting ATP synthase complex",
  "term_id": "GO:0045259"
}